intracellular cAMP-activated cation channel activity involved in regulation of postsynaptic membrane potential [GO:0140233] (molecular function) Definition: Enables the transmembrane transfer of a cation by a channel that opens when intracellular cAMP has been bound by the channel complex or one of its constituent parts, to regulate the postsynaptic membrane potential. Relationships: is a type of GO:0005222; is part of regulation of postsynaptic membrane potential [GO:0060078] Also known as: intracellular cAMP activated cation channel activity involved in regulation of postsynaptic membrane potential Note: Note that this term was created for the SynGO project, and will be obsoleted when the SynGO annotations are made in Noctua. Sources: GOC:pvn